{
  "gene_symbol": "CFC1",
  "gene_name": "Cryptic protein",
  "term_label": "blood vessel development",
  "term_id": "GO:0001568",
  "gene": "UniProtKB:P0CG37"
}